{
  "term_label": "Unknown biological process",
  "gene_symbol": "UBE2DNL",
  "gene": "UniProtKB:Q8IWF7",
  "term_id": "UNKNOWN:0002",
  "gene_name": "Putative ubiquitin-conjugating enzyme E2 D2-like protein"
}